glucuronoside transmembrane transporter activity [GO:0015164] (molecular function) Subtypes: glucuronide:cation symporter activity [GO:0015488] Also known as: glucuronide transporter activity Sources: GOC:ai, GOC:mtg_transport, ISBN:0815340729 Relationships: is a type of carbohydrate derivative transmembrane transporter activity [GO:1901505]; is part of glucuronoside transport [GO:0015779] Definition: Enables the transfer of a glucuronosides from one side of a membrane to the other. Glucuronosides are any compound formed by combination of glycosidic linkage of a hydroxy compound (e.g. an alcohol or a saccharide) with the anomeric carbon atom of glucuronate.